sucrose transmembrane transporter activity [GO:0008515] (molecular function) Sources: GOC:mtg_transport, ISBN:0198506732, ISBN:0815340729 Relationships: is a type of disaccharide transmembrane transporter activity [GO:0015154]; is part of sucrose transport [GO:0015770] Subtypes: GO:0009669, GO:0022878 Definition: Enables the transfer of sucrose from one side of a membrane to the other. Sucrose is the disaccharide O-beta-D-fructofuranosyl-(2->1)-alpha-D-glucopyranoside, a sweet-tasting, non-reducing sugar isolated industrially from sugar beet or sugar cane. Also known as: sucrose permease (PTS) activity, sucrose permease activity